{
  "gene_symbol": "SCN2A",
  "term_label": "voltage-gated sodium channel complex",
  "gene": "UniProtKB:Q99250",
  "gene_name": "Sodium channel protein type 2 subunit alpha",
  "term_id": "GO:0001518"
}